{
  "term_label": "transcription cis-regulatory region binding",
  "gene_symbol": "ZNF850",
  "term_id": "GO:0000976",
  "gene_name": "Zinc finger protein 850",
  "gene": "UniProtKB:A8MQ14"
}